regulation of angiotensin-activated signaling pathway [GO:0110061] (BP) Definition: Any process that modulates the frequency, rate or extent of the angiotensin-activated signaling pathway. Relationships: is a type of regulation of G protein-coupled receptor signaling pathway [GO:0008277]; regulates angiotensin-activated signaling pathway [GO:0038166] References: PMID:28784619 Sources: GOC:lf Subtypes: negative regulation of angiotensin-activated signaling pathway [GO:0110062], positive regulation of angiotensin-activated signaling pathway [GO:0110063]